{
  "term_label": "cytoplasm",
  "gene_name": "Peptidyl-prolyl cis-trans isomerase A-like 4E",
  "gene": "UniProtKB:A0A075B759",
  "term_id": "GO:0005737",
  "gene_symbol": "PPIAL4E"
}